{
  "gene": "UniProtKB:Q9ULJ6",
  "term_id": "GO:0061665",
  "gene_symbol": "ZMIZ1",
  "gene_name": "Zinc finger MIZ domain-containing protein 1",
  "term_label": "SUMO ligase activity"
}